subrhabdomeral cisterna [GO:0016029] (cellular component) Definition: A membrane-bounded compartment that is found at the base of the rhabdomere and contains stored calcium, InsP3 receptors and smooth endoplasmic reticulum Ca2+-ATPase. Also known as: submicrovillar cisterna, SMC References: PMID:11707492, PMID:8646774 Relationships: is a type of endoplasmic reticulum subcompartment [GO:0098827]; is a type of smooth endoplasmic reticulum cisterna [GO:0120082]; is part of GO:0016028